{
  "gene_symbol": "CDCA5",
  "gene": "UniProtKB:Q96FF9",
  "term_label": "double-strand break repair",
  "gene_name": "Sororin",
  "term_id": "GO:0006302"
}